negative regulation of protein localization to meiotic spindle pole body [GO:0140435] (biological process) References: PMID:22438582 Definition: Any process that stops, prevents or reduces the frequency, rate or extent of protein localization to a meiotic spindle pole body. Relationships: is a type of regulation of protein localization to meiotic spindle pole body [GO:0140433]; is a type of negative regulation of protein localization to spindle pole body [GO:1902364]; negatively regulates protein localization to meiotic spindle pole body [GO:1902441]